{
  "gene_symbol": "SCAPER",
  "gene": "UniProtKB:Q9BY12",
  "term_id": "UNKNOWN:0001",
  "term_label": "Unknown molecular function",
  "gene_name": "S phase cyclin A-associated protein in the endoplasmic reticulum"
}